spliceosomal tri-snRNP complex [GO:0097526] (cellular component) Relationships: is a type of GO:0097525 References: PMID:9452384 Sources: GOC:krc, GOC:pr, ISBN:0879695897 Definition: A spliceosomal snRNP complex that is formed by the association of the U4/U6 (or U4atac/U6atac) snRNP with the U5 snRNP. Subtypes: U4/U6 x U5 tri-snRNP complex [GO:0046540], U4atac/U6atac x U5 tri-snRNP complex [GO:0071009]